regulation of I-kappaB phosphorylation [GO:1903719] (biological process) Subtypes: negative regulation of I-kappaB phosphorylation [GO:1903720], positive regulation of I-kappaB phosphorylation [GO:1903721] References: PMID:23675531 Sources: GOC:TermGenie, GO_REF:0000058 Also known as: regulation of IKB phosphorylation, regulation of IkappaB phosphorylation, regulation of inhibitor of NF-kappaB phosphorylation, regulation of inhibitor of kappaB phosphorylation Definition: Any process that modulates the frequency, rate or extent of I-kappaB phosphorylation. Relationships: is a type of regulation of protein phosphorylation [GO:0001932]; regulates I-kappaB phosphorylation [GO:0007252]